{
  "gene_name": "T cell receptor beta variable 19",
  "term_id": "UNKNOWN:0001",
  "gene_symbol": "TRBV19",
  "term_label": "Unknown molecular function",
  "gene": "UniProtKB:A0A075B6N1"
}